{
  "gene_symbol": "SLC28A2",
  "term_label": "purine nucleoside transmembrane transporter activity",
  "gene": "UniProtKB:O43868",
  "gene_name": "Sodium_nucleoside cotransporter 2",
  "term_id": "GO:0015211"
}